{
  "gene": "UniProtKB:Q9BWX1",
  "gene_symbol": "PHF7",
  "term_id": "UNKNOWN:0002",
  "gene_name": "PHD finger protein 7",
  "term_label": "Unknown biological process"
}